molecular condensate scaffold activity [GO:0140693] (molecular function) References: PMID:28225081 Definition: Binding and bringing together two or more macromolecules in contact, permitting those molecules to organize as a molecular condensate. Relationships: is a type of protein-macromolecule adaptor activity [GO:0030674] Also known as: phase separation nucleation activity, phase separation nucleator activity